{
  "gene_symbol": "PRPSAP2",
  "gene": "UniProtKB:O60256",
  "gene_name": "Phosphoribosyl pyrophosphate synthase-associated protein 2",
  "term_label": "5-phosphoribose 1-diphosphate biosynthetic process",
  "term_id": "GO:0006015"
}